{
  "term_label": "negative regulation of canonical Wnt signaling pathway",
  "gene": "UniProtKB:P50402",
  "gene_symbol": "EMD",
  "gene_name": "Emerin",
  "term_id": "GO:0090090"
}